{
  "gene": "UniProtKB:P12755",
  "gene_symbol": "SKI",
  "term_id": "GO:0005667",
  "gene_name": "Ski oncogene",
  "term_label": "transcription regulator complex"
}